{
  "term_label": "DNA-(apurinic or apyrimidinic site) endonuclease activity",
  "gene_name": "DNA-(apurinic or apyrimidinic site) endonuclease",
  "gene_symbol": "APEX1",
  "term_id": "GO:0003906",
  "gene": "UniProtKB:P27695"
}